{
  "gene_symbol": "CHIT1",
  "gene": "UniProtKB:Q13231",
  "gene_name": "Chitotriosidase-1",
  "term_id": "GO:0006032",
  "term_label": "chitin catabolic process"
}